{
  "gene_symbol": "SMIM8",
  "gene_name": "Small integral membrane protein 8",
  "gene": "UniProtKB:Q96KF7",
  "term_id": "UNKNOWN:0003",
  "term_label": "Unknown cellular component"
}